{
  "gene_symbol": "DEFB130B",
  "gene": "UniProtKB:P0DP73",
  "term_id": "GO:0005615",
  "term_label": "extracellular space",
  "gene_name": "Beta-defensin 130B"
}